xylem and phloem pattern formation [GO:0010051] (biological process) Also known as: vascular tissue pattern formation Relationships: is_a regionalization [GO:0003002] Subtypes: GO:0010222, leaf vascular tissue pattern formation [GO:0010305], cotyledon vascular tissue pattern formation [GO:0010588], GO:0080056, sepal vascular tissue pattern formation [GO:0080057] Definition: The regionalization process that gives rise to the patterning of the conducting tissues. An example of this process is found in Arabidopsis thaliana. Sources: GOC:mtg_sensu, GOC:tb